{
  "gene_symbol": "CMAS",
  "term_id": "GO:0008781",
  "gene_name": "N-acylneuraminate cytidylyltransferase",
  "gene": "UniProtKB:Q8NFW8",
  "term_label": "N-acylneuraminate cytidylyltransferase activity"
}